regulation of phosphatidylserine exposure on apoptotic cell surface [GO:1905780] (biological process) References: PMID:17401362 Sources: GOC:TermGenie, GOC:kmv, GO_REF:0000058 Definition: Any process that modulates the frequency, rate or extent of phosphatidylserine exposure on apoptotic cell surface. Subtypes: GO:1905781, positive regulation of phosphatidylserine exposure on apoptotic cell surface [GO:1905782] Also known as: regulation of externalization of phosphatidylserine Relationships: is a type of regulation of phospholipid translocation [GO:0061091]; is a type of regulation of plasma membrane organization [GO:1903729]; regulates phosphatidylserine exposure on apoptotic cell surface [GO:0070782]